vascular endothelial growth factor receptor binding [GO:0005172] (molecular function) Subtypes: GO:0043183, vascular endothelial growth factor receptor 2 binding [GO:0043184], vascular endothelial growth factor receptor 3 binding [GO:0043185] Definition: Binding to a vascular endothelial growth factor receptor. Relationships: is a type of GO:0005126; is a type of growth factor receptor binding [GO:0070851] Sources: GOC:ai Also known as: VEGF receptor binding, VEGFR binding, vascular endothelial growth factor, vascular endothelial growth factor receptor ligand